{
  "term_label": "Unknown cellular component",
  "gene_symbol": "PCYOX1",
  "gene_name": "Prenylcysteine oxidase 1",
  "term_id": "UNKNOWN:0003",
  "gene": "UniProtKB:Q9UHG3"
}